positive regulation of protein localization to plasma membrane [GO:1903078] (biological process) Relationships: is a type of regulation of protein localization to plasma membrane [GO:1903076]; is a type of positive regulation of protein localization to cell periphery [GO:1904377]; is a type of positive regulation of protein localization to membrane [GO:1905477]; positively regulates protein localization to plasma membrane [GO:0072659] Subtypes: positive regulation of Golgi to plasma membrane protein transport [GO:0042998], positive regulation of endosome to plasma membrane protein transport [GO:1905751], positive regulation of protein localization to prospore membrane [GO:2001232] References: PMID:11602640 Sources: GOC:BHF, GOC:TermGenie, GOC:rl, GO_REF:0000058 Also known as: positive regulation of protein localisation in plasma membrane, positive regulation of protein localization in plasma membrane, up regulation of protein localisation in plasma membrane, up regulation of protein localization in plasma membrane, up regulation of protein localization to plasma membrane, up-regulation of protein localisation in plasma membrane, up-regulation of protein localization in plasma membrane, up-regulation of protein localization to plasma membrane, upregulation of protein localisation in plasma membrane, upregulation of protein localization in plasma membrane, upregulation of protein localization to plasma membrane, activation of protein localisation in plasma membrane, activation of protein localization in plasma membrane, activation of protein localization to plasma membrane, activation of protein targeting to plasma membrane, activation of protein-plasma membrane targeting, positive regulation of establishment of protein localisation in plasma membrane, positive regulation of establishment of protein localization to plasma membrane, positive regulation of protein targeting to plasma membrane, positive regulation of protein-plasma membrane targeting, up regulation of protein targeting to plasma membrane, up regulation of protein-plasma membrane targeting, up-regulation of protein targeting to plasma membrane, up-regulation of protein-plasma membrane targeting, upregulation of protein targeting to plasma membrane, upregulation of protein-plasma membrane targeting Definition: Any process that activates or increases the frequency, rate or extent of protein localization to plasma membrane.